{
  "gene_symbol": "PI4K2A",
  "gene_name": "Phosphatidylinositol 4-kinase type 2-alpha",
  "term_id": "GO:0046854",
  "term_label": "phosphatidylinositol phosphate biosynthetic process",
  "gene": "UniProtKB:Q9BTU6"
}